{
  "gene_symbol": "RAB38",
  "gene_name": "Ras-related protein Rab-38",
  "term_label": "endomembrane system",
  "term_id": "GO:0012505",
  "gene": "UniProtKB:P57729"
}